{
  "gene_name": "Nucleotide-binding oligomerization domain-containing protein 2",
  "term_label": "cytosol",
  "term_id": "GO:0005829",
  "gene_symbol": "NOD2",
  "gene": "UniProtKB:Q9HC29"
}